{
  "term_id": "GO:0005770",
  "gene_symbol": "TTPA",
  "gene_name": "Alpha-tocopherol transfer protein",
  "term_label": "late endosome",
  "gene": "UniProtKB:P49638"
}